{
  "gene_name": "Kinesin-like protein KIF7",
  "gene_symbol": "KIF7",
  "term_id": "GO:0003777",
  "gene": "UniProtKB:Q2M1P5",
  "term_label": "microtubule motor activity"
}